regulation of transforming growth factor beta production [GO:0071634] (BP) Subtypes: regulation of transforming growth factor beta1 production [GO:0032908], regulation of transforming growth factor beta2 production [GO:0032909], regulation of transforming growth factor beta3 production [GO:0032910], negative regulation of transforming growth factor beta production [GO:0071635], positive regulation of transforming growth factor beta production [GO:0071636] Also known as: regulation of TGF-B production, regulation of TGF-beta production, regulation of TGFB production, regulation of TGFbeta production, regulation of transforming growth factor-beta production, regulation of transforming growth factor-beta secretion Relationships: is_a GO:0001817; regulates transforming growth factor beta production [GO:0071604] Definition: Any process that modulates the frequency, rate, or extent of production of transforming growth factor-beta. Sources: GOC:mah